{
  "term_id": "GO:0043235",
  "gene_symbol": "TEK",
  "gene": "UniProtKB:Q02763",
  "gene_name": "Angiopoietin-1 receptor",
  "term_label": "receptor complex"
}